fin morphogenesis [GO:0033334] (biological process) Definition: The process in which the anatomical structures of a fin are generated and organized. Relationships: is a type of appendage morphogenesis [GO:0035107]; is part of GO:0033333 Subtypes: pectoral fin morphogenesis [GO:0035138], GO:0035139, medial fin morphogenesis [GO:0035141] Sources: GOC:dgh